{
  "term_id": "GO:0008506",
  "term_label": "sucrose:proton symporter activity",
  "gene": "UniProtKB:Q96JT2",
  "gene_symbol": "SLC45A3",
  "gene_name": "Solute carrier family 45 member 3"
}